{
  "gene_symbol": "PPARA",
  "term_label": "fatty acid metabolic process",
  "gene_name": "Peroxisome proliferator-activated receptor alpha",
  "gene": "UniProtKB:Q07869",
  "term_id": "GO:0006631"
}